{
  "gene_name": "Myb_SANT-like DNA-binding domain-containing protein 2",
  "gene_symbol": "MSANTD2",
  "term_id": "UNKNOWN:0001",
  "term_label": "Unknown molecular function",
  "gene": "UniProtKB:Q6P1R3"
}